{
  "gene": "UniProtKB:P05556",
  "gene_symbol": "ITGB1",
  "term_label": "collagen binding involved in cell-matrix adhesion",
  "term_id": "GO:0098639",
  "gene_name": "Integrin beta-1"
}